xylitol catabolic process to D-xylulose 5-phosphate [GO:0019697] (biological process) Sources: MetaCyc:LARABITOLUTIL-PWY Note: Note that xylitol is a meso compound, thus there are no L or D-versions. Also known as: L-arabitol and xylitol degradation, xylitol breakdown to xylulose 5-phosphate, xylitol degradation to xylulose 5-phosphate, xylitol utilization Definition: The chemical reactions and pathways resulting in the breakdown of xylitol to form xylulose 5-phosphate. Relationships: is a type of xylitol catabolic process [GO:0051160]; is a type of D-xylulose 5-phosphate metabolic process [GO:0051167]